cellular response to endogenous stimulus [GO:0071495] (biological process) Subtypes: GO:0003127, detection of nuclear:cytoplasmic ratio [GO:0016475], cellular response to hormone stimulus [GO:0032870], cellular response to growth factor stimulus [GO:0071363], response to cell cycle checkpoint signaling [GO:0072396] Definition: Any process that results in a change in state or activity of a cell (in terms of movement, secretion, enzyme production, gene expression, etc.) as a result of a stimulus arising within the organism. Note: Note that this term is in the subset of terms that should not be used for direct gene product annotation. Instead, select a child term or, if no appropriate child term exists, please request a new term. Direct annotations to this term may be amended during annotation QC. Sources: GOC:mah Relationships: is_a response to endogenous stimulus [GO:0009719]